{
  "term_label": "dynein intermediate chain binding",
  "gene_symbol": "DNAH6",
  "term_id": "GO:0045505",
  "gene_name": "Dynein axonemal heavy chain 6",
  "gene": "UniProtKB:Q9C0G6"
}